{
  "gene_symbol": "TMED7",
  "term_id": "UNKNOWN:0001",
  "gene_name": "Transmembrane emp24 domain-containing protein 7",
  "term_label": "Unknown molecular function",
  "gene": "UniProtKB:Q9Y3B3"
}